POZ domain binding [GO:0031208] (molecular function) Relationships: is a type of GO:0019904 Also known as: BTB domain, broad-complex, tramtrack, and bric-a-brac domain binding References: PMID:7958847 Definition: Binding to a POZ (poxvirus and zinc finger) domain of a protein, a protein-protein interaction domain found in many transcription factors.